leukotriene B4 catabolic process [GO:0036101] (biological process) References: PMID:9799565 Sources: GOC:yaf Definition: The chemical reactions and pathways resulting in the breakdown of leukotriene B4, a leukotriene composed of (6Z,8E,10E,14Z)-eicosatetraenoic acid having (5S)- and (12R)-hydroxy substituents. Relationships: is a type of leukotriene catabolic process [GO:0036100]; is a type of leukotriene B4 metabolic process [GO:0036102]; is a type of long-chain fatty acid catabolic process [GO:0042758]; is a type of icosanoid catabolic process [GO:1901523] Also known as: LTB4 catabolism, leukotriene B4 breakdown, leukotriene B4 catabolism, leukotriene B4 degradation